{
  "gene_symbol": "PSMC2",
  "term_label": "proteasome regulatory particle, base subcomplex",
  "gene_name": "26S proteasome regulatory subunit 7",
  "gene": "UniProtKB:P35998",
  "term_id": "GO:0008540"
}